{
  "gene_symbol": "ATXN7L3",
  "gene_name": "Ataxin-7-like protein 3",
  "term_label": "transcription coactivator activity",
  "gene": "UniProtKB:Q14CW9",
  "term_id": "GO:0003713"
}